cortical cytoskeleton [GO:0030863] (CC) Relationships: is a type of GO:0005856; is part of GO:0005938 Sources: GOC:mah Subtypes: cortical actin cytoskeleton [GO:0030864], GO:0030981, cytoskeleton of presynaptic active zone [GO:0048788] Definition: The portion of the cytoskeleton that lies just beneath the plasma membrane.